regulation of cholesterol biosynthetic process [GO:0045540] (biological process) Relationships: is a type of regulation of cholesterol metabolic process [GO:0090181]; is a type of GO:0106118; is a type of regulation of alcohol biosynthetic process [GO:1902930]; regulates GO:0006695 Also known as: regulation of cholesterol anabolism, regulation of cholesterol biosynthesis, regulation of cholesterol formation, regulation of cholesterol synthesis Definition: Any process that modulates the frequency, rate or extent of the chemical reactions and pathways resulting in the formation of cholesterol. Sources: GOC:go_curators Subtypes: negative regulation of cholesterol biosynthetic process [GO:0045541], positive regulation of cholesterol biosynthetic process [GO:0045542]